{
  "gene_name": "Type III endosome membrane protein TEMP",
  "gene_symbol": "C1orf210",
  "term_id": "UNKNOWN:0002",
  "gene": "UniProtKB:Q8IVY1",
  "term_label": "Unknown biological process"
}